{
  "gene_name": "Exocyst complex component 6",
  "gene": "UniProtKB:Q8TAG9",
  "gene_symbol": "EXOC6",
  "term_id": "UNKNOWN:0001",
  "term_label": "Unknown molecular function"
}